{
  "term_label": "cytosol",
  "term_id": "GO:0005829",
  "gene": "UniProtKB:O95336",
  "gene_name": "6-phosphogluconolactonase",
  "gene_symbol": "PGLS"
}